mitochondrial cloud [GO:0032019] (cellular component) Definition: A prominent mass in the cytoplasm of previtellogenic oocytes. The cloud contains both mitochondria and electron-dense granulofibrillar material (GFM) and is the source of germinal granule material. Also known as: Balbiani body, mitochondrial aggregate Relationships: is a type of intracellular membraneless organelle [GO:0043232]; is part of cytoplasm [GO:0005737] References: PMID:6541166